regulation of eosinophil migration [GO:2000416] (biological process) Sources: GOC:mah Relationships: is a type of regulation of leukocyte migration [GO:0002685]; regulates GO:0072677 Definition: Any process that modulates the frequency, rate or extent of eosinophil migration. Subtypes: negative regulation of eosinophil migration [GO:2000417], GO:2000418, regulation of eosinophil extravasation [GO:2000419], regulation of eosinophil chemotaxis [GO:2000422]